{
  "gene_name": "Aurora kinase C",
  "gene": "UniProtKB:Q9UQB9",
  "term_label": "midbody",
  "term_id": "GO:0030496",
  "gene_symbol": "AURKC"
}